{
  "gene": "UniProtKB:O14829",
  "term_label": "Unknown biological process",
  "gene_symbol": "PPEF1",
  "gene_name": "Serine_threonine-protein phosphatase with EF-hands 1",
  "term_id": "UNKNOWN:0002"
}